RQC complex [GO:1990112] (cellular component) Also known as: ribosome quality control complex, ribosome-bound quality control complex Relationships: is a type of protein-containing complex [GO:0032991] Definition: A multiprotein complex that forms a stable complex with large ribosomal subunits (60S in eukaryotes and 50S in prokaryotes) containing stalled polypeptides and triggers their degradation (ribosomal quality control). In budding yeast, this complex includes Cdc48p, Rkr1p, Tae2p, Rqc1p, Npl4p and Ufd1p proteins. References: PMID:23178123, PMID:23232563 Sources: GOC:rb